{
  "gene": "UniProtKB:P0C7M8",
  "gene_name": "C-type lectin domain family 2 member L",
  "term_label": "Unknown cellular component",
  "gene_symbol": "CLEC2L",
  "term_id": "UNKNOWN:0003"
}